{
  "gene": "UniProtKB:Q9UPN6",
  "term_label": "mRNA binding",
  "gene_symbol": "SCAF8",
  "gene_name": "SR-related and CTD-associated factor 8",
  "term_id": "GO:0003729"
}